positive regulation of hippo signaling [GO:0035332] (biological process) Relationships: is a type of regulation of hippo signaling [GO:0035330]; is a type of positive regulation of intracellular signal transduction [GO:1902533]; positively regulates hippo signaling [GO:0035329] Sources: GOC:bf Also known as: positive regulation of hippo signaling pathway, positive regulation of hippo signaling cascade, positive regulation of hippo signalling cascade Definition: Any process that activates or increases the frequency, rate or extent of hippo signaling.